{
  "term_id": "GO:0032266",
  "term_label": "phosphatidylinositol-3-phosphate binding",
  "gene_symbol": "TECPR1",
  "gene": "UniProtKB:Q7Z6L1",
  "gene_name": "Tectonin beta-propeller repeat-containing protein 1"
}